{
  "gene_symbol": "SLC12A9",
  "term_id": "GO:0006884",
  "gene_name": "Solute carrier family 12 member 9",
  "gene": "UniProtKB:Q9BXP2",
  "term_label": "cell volume homeostasis"
}